helicase activity [GO:0004386] (molecular function) Relationships: is a type of nucleic acid conformation isomerase activity [GO:0120545]; is a type of catalytic activity, acting on a nucleic acid [GO:0140640]; is a type of ATP-dependent activity [GO:0140657] Note: Note that most helicases catalyze processive duplex unwinding. Definition: Catalysis of the reaction: ATP + H2O = ADP + phosphate, to drive the unwinding of a DNA or RNA helix. Sources: GOC:jl Subtypes: DNA helicase activity [GO:0003678], RNA helicase activity [GO:0003724], DNA/RNA helicase activity [GO:0033677] Regulation: positively regulated by positive regulation of helicase activity [GO:0051096]; negatively regulated by negative regulation of helicase activity [GO:0051097] Also known as: ATP-dependent helicase activity